translation [GO:0006412] (BP) Subtypes: cytoplasmic translation [GO:0002181], GO:0032543, plastid translation [GO:0032544], translation at synapse [GO:0140241] Definition: The cellular metabolic process in which a protein is formed, using the sequence of a mature mRNA or circRNA molecule to specify the sequence of amino acids in a polypeptide chain. Translation is mediated by the ribosome, and begins with the formation of a ternary complex between aminoacylated initiator methionine tRNA, GTP, and initiation factor 2, which subsequently associates with the small subunit of the ribosome and an mRNA or circRNA. Translation ends with the release of a polypeptide chain from the ribosome. Sources: GOC:go_curators Regulation: regulated by GO:0006417; negatively regulated by negative regulation of translation [GO:0017148]; RO_0002213 by GO:0045727 Relationships: is a type of GO:0009059; is a type of protein metabolic process [GO:0019538]; is part of protein biosynthetic process [GO:0160307]; has part GO:0000048; has part GO:0006413; has part translational elongation [GO:0006414]; has part GO:0006415 Also known as: protein translation